{
  "term_label": "intermediate filament",
  "gene_name": "Filensin",
  "gene": "UniProtKB:Q12934",
  "term_id": "GO:0005882",
  "gene_symbol": "BFSP1"
}